{
  "term_id": "UNKNOWN:0003",
  "gene_symbol": "LYPD2",
  "gene_name": "Ly6_PLAUR domain-containing protein 2",
  "term_label": "Unknown cellular component",
  "gene": "UniProtKB:Q6UXB3"
}